{
  "term_label": "SCF-dependent proteasomal ubiquitin-dependent protein catabolic process",
  "gene_name": "F-box only protein 44",
  "term_id": "GO:0031146",
  "gene_symbol": "FBXO44",
  "gene": "UniProtKB:Q9H4M3"
}